{
  "gene": "UniProtKB:P49619",
  "term_id": "GO:0006654",
  "term_label": "phosphatidic acid biosynthetic process",
  "gene_name": "Diacylglycerol kinase gamma",
  "gene_symbol": "DGKG"
}